anterior/posterior axis specification, embryo [GO:0008595] (biological process) Relationships: is a type of embryonic axis specification [GO:0000578]; is a type of anterior/posterior axis specification [GO:0009948]; is part of tripartite regional subdivision [GO:0007351] Sources: ISBN:0879694238, http://fly.ebi.ac.uk/allied-data/lk/interactive-fly/aimain/1aahome.htm Definition: The specification of the anterior/posterior axis of the embryo by the products of genes expressed maternally and genes expressed in the zygote. Also known as: anterior/posterior axis determination, embryo Subtypes: zygotic determination of anterior/posterior axis, embryo [GO:0007354], maternal determination of anterior/posterior axis, embryo [GO:0008358]